regulation of synaptic activity [GO:0060025] (biological process) Relationships: is a type of modulation of chemical synaptic transmission [GO:0050804]; is part of regulation of synapse structure or activity [GO:0050803] Definition: Any process that modulates the frequency, rate or extent of synaptic activity, the controlled release of neurotransmitters into the synaptic cleft and their subsequent detection by a postsynaptic cell. Sources: GOC:dph, GOC:tb